{
  "gene_symbol": "GAL3ST2",
  "gene_name": "Galactose-3-O-sulfotransferase 2",
  "term_label": "Unknown cellular component",
  "gene": "UniProtKB:Q9H3Q3",
  "term_id": "UNKNOWN:0003"
}